{
  "term_id": "UNKNOWN:0001",
  "gene": "UniProtKB:Q96R06",
  "gene_name": "Sperm-associated antigen 5",
  "gene_symbol": "SPAG5",
  "term_label": "Unknown molecular function"
}